intracellular signaling cassette [GO:0141124] (biological process) Relationships: is a type of intracellular signal transduction [GO:0035556] Definition: An intracellular signaling module that is part of larger signaling pathways that can be initiated either intracellularly or by cell surface receptors. Intracellular signaling cassettes are discrete signaling units that are often shared by multiple signaling pathways. Subtypes: GO:0000165, canonical NF-kappaB signal transduction [GO:0007249], nitric oxide mediated signal transduction [GO:0007263], GO:0007264, calcium-mediated signaling [GO:0019722], non-canonical NF-kappaB signal transduction [GO:0038061], phosphatidylinositol 3-kinase/protein kinase B signal transduction [GO:0043491], GO:0060395, GO:0140467, cAMP/PKA signal transduction [GO:0141156], GO:0141212 Sources: GOC:ha, GOC:pg Also known as: intracellular signaling cascade, intracellular signaling module